H4 histamine receptor binding [GO:0031810] (molecular function) Sources: GOC:mah, GOC:nln Also known as: H4 histamine receptor ligand Definition: Binding to a H4 histamine receptor. Relationships: is a type of G protein-coupled histamine receptor binding [GO:0031806]